central canal development [GO:0061524] (biological process) Definition: The process whose specific outcome is the formation of the central canal of the spinal cord from its formation to the mature structure. The central canal is a spinal cord structure that is part of the ventricular system and is filled with cerebral-spinal fluid and runs the length of the spinal cord. References: PMID:23409159 Sources: GOC:cvs, GOC:dph Relationships: is a type of anatomical structure development [GO:0048856]; is part of spinal cord development [GO:0021510]